negative regulation of heart rate involved in baroreceptor response to increased systemic arterial blood pressure [GO:0001985] (BP) Definition: Any process that stops, prevents, or reduces the frequency, rate or extent of heart contraction as a result of the baroreceptor response to increased blood pressure. Relationships: is a type of negative regulation of heart rate [GO:0010459]; is part of baroreceptor response to increased systemic arterial blood pressure [GO:0001983] Sources: ISBN:0721643949 Also known as: down regulation of heart contraction rate in baroreceptor response to increased blood pressure, down-regulation of heart contraction rate in baroreceptor response to increased blood pressure, downregulation of heart contraction rate in baroreceptor response to increased blood pressure, negative control of heart contraction rate in baroreceptor response to increased blood pressure, negative regulation of heart contraction rate in baroreceptor response to increased blood pressure, inhibition of heart contraction rate in baroreceptor response to increased blood pressure, negative regulation of cardiac contraction rate in baroreceptor response to increased blood pressure